{
  "gene_name": "Phospholipid-transporting ATPase ABCA1",
  "gene": "UniProtKB:O95477",
  "term_label": "phospholipid efflux",
  "term_id": "GO:0033700",
  "gene_symbol": "ABCA1"
}